{
  "term_id": "GO:0030424",
  "gene_name": "Actin-like protein 8",
  "term_label": "axon",
  "gene": "UniProtKB:Q9H568",
  "gene_symbol": "ACTL8"
}